positive regulation of hemicellulose catabolic process [GO:2000990] (biological process) Also known as: positive regulation of hemicellulose catabolism Sources: GOC:mengo_curators Definition: Any process that activates or increases the frequency, rate or extent of hemicellulose catabolic process. Subtypes: positive regulation of xyloglucan catabolic process [GO:2000953], positive regulation of xylan catabolic process [GO:2001002] Relationships: is a type of positive regulation of catabolic process [GO:0009896]; is a type of positive regulation of macromolecule metabolic process [GO:0010604]; is a type of positive regulation of carbohydrate metabolic process [GO:0045913]; is a type of regulation of hemicellulose catabolic process [GO:2000988]; positively regulates hemicellulose catabolic process [GO:2000895]